{
  "term_id": "GO:0005741",
  "gene": "UniProtKB:Q8IXI2",
  "gene_symbol": "RHOT1",
  "term_label": "mitochondrial outer membrane",
  "gene_name": "Mitochondrial Rho GTPase 1"
}